negative regulation of developmental pigmentation [GO:0048086] (biological process) Sources: GOC:dph, GOC:jid, GOC:tb Relationships: is a type of regulation of developmental pigmentation [GO:0048070]; is a type of negative regulation of biological process [GO:0048519]; negatively regulates GO:0048066 Also known as: down regulation of developmental pigmentation, down-regulation of developmental pigmentation, downregulation of developmental pigmentation, inhibition of pigmentation Definition: Any process that decreases the frequency, rate or extent of the developmental process that results in the deposition of coloring matter in an organism. Subtypes: negative regulation of eye pigmentation [GO:0048074], GO:0048080, GO:0048090, negative regulation of male pigmentation [GO:0048092], GO:0050941